{
  "gene_symbol": "HNRNPCL2",
  "gene": "UniProtKB:B2RXH8",
  "term_label": "nucleus",
  "term_id": "GO:0005634",
  "gene_name": "Heterogeneous nuclear ribonucleoprotein C-like 2"
}